{
  "gene_symbol": "HOMER2",
  "term_label": "sensory perception of sound",
  "term_id": "GO:0007605",
  "gene_name": "Homer protein homolog 2",
  "gene": "UniProtKB:Q9NSB8"
}